regulation of pattern recognition receptor signaling pathway [GO:0062207] (BP) Definition: Any process that modulates the rate, frequency or extent of a pattern recognition receptor signaling pathway. Relationships: is a type of GO:0009966; is a type of regulation of innate immune response [GO:0045088]; regulates pattern recognition receptor signaling pathway [GO:0002221] References: PMID:30610168 Subtypes: regulation of toll-like receptor signaling pathway [GO:0034121], GO:0034131, regulation of toll-like receptor 2 signaling pathway [GO:0034135], regulation of toll-like receptor 4 signaling pathway [GO:0034143], GO:0034147, GO:0034151, regulation of toll-like receptor 10 signaling pathway [GO:0034167], regulation of cytoplasmic pattern recognition receptor signaling pathway [GO:0039531], regulation of peptidoglycan recognition protein signaling pathway [GO:0061058], positive regulation of pattern recognition receptor signaling pathway [GO:0062208], regulation of toll-like receptor 15 signaling pathway [GO:2000440]